positive regulation of calcium-dependent cell-cell adhesion [GO:0046587] (biological process) Relationships: is a type of positive regulation of cell-cell adhesion [GO:0022409]; is a type of GO:0046586; RO_0002213 GO:0016339 Sources: GOC:ai Also known as: up regulation of calcium-dependent cell-cell adhesion, up-regulation of calcium-dependent cell-cell adhesion, upregulation of calcium-dependent cell-cell adhesion, activation of calcium-dependent cell-cell adhesion, stimulation of calcium-dependent cell-cell adhesion Definition: Any process that activates or increases the frequency, rate or extent of calcium-dependent cell-cell adhesion.